{
  "term_label": "Unknown cellular component",
  "gene_symbol": "PMCHL1",
  "term_id": "UNKNOWN:0003",
  "gene": "UniProtKB:Q16048",
  "gene_name": "Putative pro-MCH-like protein 1"
}